{
  "term_label": "Unknown molecular function",
  "gene_name": "Ciliogenesis-associated TTC17-interacting protein",
  "gene": "UniProtKB:Q7Z7H3",
  "term_id": "UNKNOWN:0001",
  "gene_symbol": "CATIP"
}